{
  "gene_symbol": "PTBP2",
  "gene": "UniProtKB:Q9UKA9",
  "term_label": "regulation of RNA splicing",
  "gene_name": "Polypyrimidine tract-binding protein 2",
  "term_id": "GO:0043484"
}